somato-dendritic dopamine secretion [GO:0099123] (biological process) Also known as: STD DA release, STD dopamine release, somatodendritic dopamine release Definition: The regulated release of dopamine from the somatodendritic compartment (cell body or dendrites) of a neuron. Relationships: is a type of dopamine secretion [GO:0014046]; is a type of establishment of localization in cell [GO:0051649]; occurs in somatodendritic compartment [GO:0036477] References: PMID:21576241 Sources: GOC:PARL, GOC:bf